{
  "term_id": "GO:0006888",
  "term_label": "endoplasmic reticulum to Golgi vesicle-mediated transport",
  "gene": "UniProtKB:Q13190",
  "gene_name": "Syntaxin-5",
  "gene_symbol": "STX5"
}